telomere maintenance via semi-conservative replication [GO:0032201] (biological process) Definition: The process in which telomeric DNA is synthesized semi-conservatively by the conventional replication machinery and telomeric accessory factors as part of cell cycle DNA replication. Subtypes: meiotic telomere maintenance via semi-conservative replication [GO:1902989], mitotic telomere maintenance via semi-conservative replication [GO:1902990] Relationships: is a type of GO:0000723; is a type of cell cycle process [GO:0022402]; is part of nuclear DNA replication [GO:0033260] References: PMID:16598261 Sources: GOC:BHF, GOC:BHF_telomere, GOC:rl, GOC:vw Regulation: regulated by GO:0032213; negatively regulated by GO:0032214; positively regulated by GO:0032215 Also known as: telomeric fork progression, telomeric replication fork progression, equal telomere replication